{
  "term_id": "UNKNOWN:0002",
  "gene": "UniProtKB:P0C7V4",
  "gene_name": "Putative protein FAM90A15P",
  "gene_symbol": "FAM90A15P",
  "term_label": "Unknown biological process"
}